{
  "gene": "UniProtKB:P59817",
  "term_id": "GO:0000978",
  "gene_name": "Zinc finger protein 280A",
  "term_label": "RNA polymerase II cis-regulatory region sequence-specific DNA binding",
  "gene_symbol": "ZNF280A"
}